{
  "term_id": "GO:0042571",
  "term_label": "immunoglobulin complex, circulating",
  "gene_symbol": "IGHG3",
  "gene_name": "Immunoglobulin heavy constant gamma 3",
  "gene": "UniProtKB:P01860"
}